{
  "gene_symbol": "ZNF335",
  "gene_name": "Zinc finger protein 335",
  "gene": "UniProtKB:Q9H4Z2",
  "term_id": "GO:0005634",
  "term_label": "nucleus"
}